{
  "gene_symbol": "GIN1",
  "gene_name": "Gypsy retrotransposon integrase-like protein 1",
  "term_label": "Unknown cellular component",
  "gene": "UniProtKB:Q9NXP7",
  "term_id": "UNKNOWN:0003"
}